{
  "gene": "UniProtKB:Q02747",
  "gene_symbol": "GUCA2A",
  "gene_name": "Guanylin",
  "term_label": "guanylate cyclase activator activity",
  "term_id": "GO:0030250"
}